{
  "gene_symbol": "Q9H3A6",
  "term_label": "Unknown cellular component",
  "gene": "UniProtKB:Q9H3A6",
  "term_id": "UNKNOWN:0003",
  "gene_name": "PRO2179"
}